{
  "term_label": "cilium",
  "term_id": "GO:0005929",
  "gene": "UniProtKB:P20794",
  "gene_symbol": "MAK",
  "gene_name": "Serine_threonine-protein kinase MAK"
}